regulation of mitotic actomyosin contractile ring assembly [GO:1903499] (BP) Also known as: regulation of actomyosin contractile ring assembly involved in cytokinesis after mitosis, regulation of contractile ring assembly involved in mitotic cytokinesis, regulation of cytokinesis, actomyosin contractile ring assembly involved in mitotic cytokinesis, regulation of mitotic cytokinesis, actomyosin contractile ring assembly Relationships: is a type of GO:1903436; is a type of regulation of cytokinesis, actomyosin contractile ring assembly [GO:2000431]; RO_0002211 GO:1903475 References: PMID:18256290 Sources: GOC:TermGenie, GOC:al, GOC:mtg_cell_cycle, GOC:vw, GO_REF:0000058 Definition: Any process that modulates the frequency, rate or extent of mitotic actomyosin contractile ring assembly. Subtypes: negative regulation of mitotic actomyosin contractile ring assembly [GO:1903500], positive regulation of mitotic actomyosin contractile ring assembly [GO:1903501]